{
  "term_id": "GO:0006357",
  "gene_symbol": "ZNF169",
  "term_label": "regulation of transcription by RNA polymerase II",
  "gene": "UniProtKB:Q14929",
  "gene_name": "Zinc finger protein 169"
}